TRAPP complex [GO:0030008] (cellular component) References: PMID:22669257 Sources: GOC:bhm, GOC:vw Definition: A large complex that acts as a tethering factor involved in transporting vesicles from the ER through the Golgi to the plasma membrane. A TRAPP (transport protein particle) complex has a core set of proteins which are joined by specific subunits depending on the cellular component where a given TRAPP complex is active. Also known as: transport protein particle, transport protein particle complex, TRAPP1, TRAPP2 Relationships: is a type of vesicle tethering complex [GO:0099023]; is_a intracellular protein-containing complex [GO:0140535] Subtypes: TRAPPI protein complex [GO:1990070], GO:1990071, GO:1990072